eosinophil homeostasis [GO:1990959] (biological process) References: PMID:10606160 Relationships: is a type of leukocyte homeostasis [GO:0001776]; is a type of GO:0002262 Also known as: eosinocyte homeostasis, eosinophilic granulocyte homeostasis, eosinophilic leucocyte homeostasis, eosinophilic leukocyte homeostasis Definition: The process of regulating the proliferation and elimination of eosinophils such that the total number of eosinophils within a whole or part of an organism is stable over time in the absence of an outside stimulus.